collectin receptor activity [GO:0001863] (molecular function) Sources: GOC:add, GOC:signaling, ISBN:0781735149 Note: Note that collectins include such proteins as mannose-binding lectin (MBL) and surfactant proteins A and D (SP-A and SP-D). Relationships: is a type of opsonin receptor activity [GO:0001847]; has part GO:0001862 Definition: Combining with a collectin and transmitting the signal from one side of the membrane to the other to initiate a change in cell activity.